{
  "gene_symbol": "HSFX2",
  "term_id": "GO:0000978",
  "gene": "UniProtKB:Q9UBD0",
  "gene_name": "Heat shock transcription factor, X-linked",
  "term_label": "RNA polymerase II cis-regulatory region sequence-specific DNA binding"
}